activin complex [GO:0048180] (cellular component) Definition: A nonsteroidal regulator, composed of two covalently linked inhibin beta subunits, inhibin beta-A and inhibin beta-B (sometimes known as activin beta or activin/inhibin beta). There are three forms of activin complex, activin A, which is composed of 2 inhibin beta-A subunits, activin B, which is composed of 2 inhibin beta-B subunits, and activin AB, which is composed of an inhibin beta-A and an inhibin beta-B subunit. Note: Note that the actions of the activin complex are the opposite of those of the inhibin complex, which is a dimer of an inhibin beta-A or inhibin beta-B subunit and a inhibin alpha subunit. See 'inhibin complex ; GO:0043511'. Sources: GOC:go_curators Subtypes: GO:0043509, activin B complex [GO:0043510], GO:0048183 Relationships: is a type of protein-containing complex [GO:0032991]; BFO_0000050 extracellular space [GO:0005615]